{
  "term_id": "GO:0007097",
  "gene_name": "Nesprin-1",
  "gene": "UniProtKB:Q8NF91",
  "term_label": "nuclear migration",
  "gene_symbol": "SYNE1"
}